pyruvate dehydrogenase (acetyl-transferring) activity [GO:0004739] (molecular function) Also known as: pyruvate dehydrogenase (lipoamide) activity, MtPDC (mitochondrial pyruvate dehydogenase complex) activity, PDH, pyruvate dehydrogenase complex activity, pyruvate:dihydrolipoyllysine-residue acetyltransferase-lipoyllysine 2-oxidoreductase (decarboxylating, acceptor-acetylating), pyruvate:lipoamide 2-oxidoreductase (decarboxylating and acceptor-acetylating) activity Definition: Catalysis of the reaction: N(6)-[(R)-lipoyl]-L-lysyl-[protein] + pyruvate + H+ = N(6)-[(R)-S(8)-acetyldihydrolipoyl]-L-lysyl-[protein] + CO2. Sources: RHEA:19189 Relationships: is a type of oxidoreductase activity, acting on the aldehyde or oxo group of donors, disulfide as acceptor [GO:0016624]